{
  "gene_symbol": "LRRC3C",
  "gene_name": "Leucine-rich repeat-containing protein 3C",
  "gene": "UniProtKB:A6NJW4",
  "term_label": "plasma membrane",
  "term_id": "GO:0005886"
}